{
  "term_label": "osteoblast development",
  "gene_symbol": "PTHLH",
  "term_id": "GO:0002076",
  "gene_name": "Parathyroid hormone-related protein",
  "gene": "UniProtKB:P12272"
}